axon guidance receptor activity [GO:0008046] (molecular function) References: PMID:15107857, PMID:15339666 Sources: GOC:dph, GOC:signaling, GOC:tb Definition: Combining with an extracellular messenger and transmitting the signal from one side of the membrane to the other to results in a change in cellular activity involved in axon guidance. Also known as: receptor activity involved in axon guidance Relationships: is a type of transmembrane signaling receptor activity [GO:0004888]; is part of axon guidance [GO:0007411]